{
  "gene_symbol": "LMO4",
  "term_id": "GO:0003712",
  "gene_name": "LIM domain transcription factor LMO4",
  "term_label": "transcription coregulator activity",
  "gene": "UniProtKB:P61968"
}